mitotic anaphase B [GO:0000092] (biological process) Note: Note that this term should not be used for direct annotation. If you are trying to make an annotation to x phase, it is likely that the correct annotation is 'regulation of x/y phase transition' or to a process which occurs during the reported phase (i.e mitotic DNA replication for mitotic S-phase). To capture the phase when a specific location or process is observed, the phase term can be used in an annotation extension (PMID:24885854) applied to a cellular component term (with the relation exists_during) or a biological process term (with the relation happens_during). Relationships: is_a GO:0000090 Definition: The cell cycle phase during which the polar microtubules elongate and the two poles of the spindle move farther apart as part of mitosis. Sources: GOC:mtg_cell_cycle